{
  "gene_symbol": "CAPN14",
  "term_id": "GO:0005737",
  "gene_name": "Calpain-14",
  "gene": "UniProtKB:A8MX76",
  "term_label": "cytoplasm"
}